response to interleukin-6 [GO:0070741] (biological process) Relationships: is a type of GO:0034097 Sources: GOC:mah Also known as: response to IL-6 Subtypes: cellular response to interleukin-6 [GO:0071354] Definition: Any process that results in a change in state or activity of a cell or an organism (in terms of movement, secretion, enzyme production, gene expression, etc.) as a result of an interleukin-6 stimulus.